catechol-containing compound biosynthetic process [GO:0009713] (biological process) Also known as: catechol anabolism, catechol biosynthesis, catechol biosynthetic process, catechol formation, catechol synthesis Subtypes: GO:0019540, (R)-mandelate catabolic process to catechol [GO:0019598], catecholamine biosynthetic process [GO:0042423], chrysobactin biosynthetic process [GO:0042858], methylgallate biosynthetic process [GO:0046277], GO:0046279, alkyl caffeate ester biosynthetic process [GO:0090431], gerfelin biosynthetic process [GO:1900578], violaceol I biosynthetic process [GO:1900590], GO:1900593, GO:1900799, 3-chlorocatechol biosynthetic process [GO:1901169], 3-(2,3-dihydroxyphenyl)propanoate biosynthetic process [GO:1901792] Sources: GOC:go_curators Definition: The chemical reactions and pathways resulting in the formation of catechol-containing compounds. Catechol is a compound containing a pyrocatechol nucleus or substituent. Relationships: is a type of catechol-containing compound metabolic process [GO:0009712]; is a type of phenol-containing compound biosynthetic process [GO:0046189]